{
  "gene_name": "Elongin BC and Polycomb repressive complex 2-associated protein",
  "term_id": "UNKNOWN:0001",
  "gene": "UniProtKB:A6NHQ4",
  "term_label": "Unknown molecular function",
  "gene_symbol": "EPOP"
}